{
  "term_id": "UNKNOWN:0001",
  "term_label": "Unknown molecular function",
  "gene_symbol": "TRAV34",
  "gene": "UniProtKB:A0A0B4J273",
  "gene_name": "T cell receptor alpha variable 34"
}